{
  "gene_name": "DNA repair protein XRCC2",
  "gene_symbol": "XRCC2",
  "gene": "UniProtKB:O43543",
  "term_label": "four-way junction DNA binding",
  "term_id": "GO:0000400"
}